lymph vessel development [GO:0001945] (biological process) Relationships: is a type of anatomical structure development [GO:0048856]; is part of vasculature development [GO:0001944] Definition: The process whose specific outcome is the progression of a lymph vessel over time, from its formation to the mature structure. Sources: GOC:dph, UBERON:0001473